{
  "gene": "UniProtKB:Q96NR8",
  "term_label": "Unknown biological process",
  "term_id": "UNKNOWN:0002",
  "gene_symbol": "RDH12",
  "gene_name": "Retinol dehydrogenase 12"
}